hypophysis formation [GO:0048851] (biological process) Sources: GOC:cls, GOC:dgh, GOC:dph, GOC:jid Relationships: is a type of anatomical structure formation involved in morphogenesis [GO:0048646]; is part of GO:0048850 Definition: The process in which the anatomical structures of the hypophysis are generated and organized. The hypophysis is an endocrine gland that secretes hormones that regulate many other glands. Also known as: hypophysis biosynthesis, pituitary gland biosynthesis, pituitary gland formation